{
  "gene_name": "E3 ubiquitin-protein ligase Topors",
  "term_id": "GO:0032391",
  "gene_symbol": "TOPORS",
  "term_label": "photoreceptor connecting cilium",
  "gene": "UniProtKB:Q9NS56"
}